{
  "term_id": "GO:0005634",
  "gene_symbol": "PWWP3A",
  "gene": "UniProtKB:Q2TAK8",
  "gene_name": "PWWP domain-containing DNA repair factor 3A",
  "term_label": "nucleus"
}